{
  "gene": "UniProtKB:Q9Y4C8",
  "gene_symbol": "RBM19",
  "term_id": "GO:0005730",
  "gene_name": "Probable RNA-binding protein 19",
  "term_label": "nucleolus"
}